{
  "term_id": "GO:0019005",
  "term_label": "SCF ubiquitin ligase complex",
  "gene": "UniProtKB:Q8NI29",
  "gene_name": "F-box only protein 27",
  "gene_symbol": "FBXO27"
}